{
  "term_label": "positive regulation of transcription by RNA polymerase II",
  "gene_symbol": "SRY",
  "gene_name": "Sex-determining region Y protein",
  "term_id": "GO:0045944",
  "gene": "UniProtKB:Q05066"
}